response to laminar fluid shear stress [GO:0034616] (biological process) Sources: GOC:ecd Definition: Any process that results in a change in state or activity of a cell or an organism (in terms of movement, secretion, enzyme production, gene expression, etc.) as a result of a laminar fluid shear stress stimulus. Laminar fluid flow is the force acting on an object in a system where the fluid is moving across a solid surface in parallel layers. As an example, laminar shear stress can be seen where blood flows against the luminal side of blood vessel walls. Relationships: is a type of response to fluid shear stress [GO:0034405] Subtypes: GO:0071499